{
  "gene": "UniProtKB:Q9NQL2",
  "gene_name": "Ras-related GTP-binding protein D",
  "term_id": "GO:1990131",
  "term_label": "Gtr1-Gtr2 GTPase complex",
  "gene_symbol": "RRAGD"
}